{
  "gene_symbol": "C17orf98",
  "term_id": "UNKNOWN:0001",
  "gene_name": "Uncharacterized protein C17orf98",
  "gene": "UniProtKB:A8MV24",
  "term_label": "Unknown molecular function"
}